{
  "gene_symbol": "IGFLR1",
  "term_label": "plasma membrane",
  "term_id": "GO:0005886",
  "gene": "UniProtKB:Q9H665",
  "gene_name": "IGF-like family receptor 1"
}